dTMP salvage [GO:0036198] (biological process) Relationships: is a type of dTMP biosynthetic process [GO:0006231]; is a type of GO:0010139 Definition: Any process which produces dTMP, deoxyribosylthymine monophosphate (2'-deoxyribosylthymine 5'-phosphate) without de novo synthesis. Also known as: dTMP biosynthesis via salvage pathway, deoxythymidine monophosphate biosynthesis via salvage pathway References: PMID:5387459 Sources: GOC:yaf